{
  "term_id": "GO:0005829",
  "gene": "UniProtKB:Q53GT1",
  "gene_symbol": "KLHL22",
  "gene_name": "Kelch-like protein 22",
  "term_label": "cytosol"
}